{
  "term_id": "UNKNOWN:0001",
  "gene_name": "Spermatogenesis-associated protein 7",
  "gene_symbol": "SPATA7",
  "gene": "UniProtKB:Q9P0W8",
  "term_label": "Unknown molecular function"
}